{
  "term_label": "Unknown biological process",
  "term_id": "UNKNOWN:0002",
  "gene": "UniProtKB:Q9Y5B8",
  "gene_name": "Nucleoside diphosphate kinase 7",
  "gene_symbol": "NME7"
}